{
  "term_label": "structural constituent of skin epidermis",
  "gene_symbol": "KRT82",
  "gene_name": "Keratin, type II cuticular Hb2",
  "term_id": "GO:0030280",
  "gene": "UniProtKB:Q9NSB4"
}